{
  "gene_symbol": "CLCC1",
  "term_label": "endoplasmic reticulum",
  "gene_name": "Chloride channel CLIC-like protein 1",
  "term_id": "GO:0005783",
  "gene": "UniProtKB:Q96S66"
}